{
  "gene_symbol": "LRP1",
  "gene_name": "Prolow-density lipoprotein receptor-related protein 1",
  "gene": "UniProtKB:Q07954",
  "term_label": "cargo receptor activity",
  "term_id": "GO:0038024"
}